virus coreceptor activity [GO:0120274] (molecular function) Also known as: viral coreceptor activity Definition: Combining with a virus component, and in cooperation with a nearby primary receptor, initiating a change in cell activity. References: PMID:16051304 Sources: GOC:ha, GOC:krc Relationships: is a type of exogenous protein binding [GO:0140272]; is part of symbiont entry into host cell [GO:0046718]